regulation of macromolecule biosynthetic process [GO:0010556] (biological process) Definition: Any process that modulates the rate, frequency or extent of the chemical reactions and pathways resulting in the formation of a macromolecule, any molecule of high relative molecular mass, the structure of which essentially comprises the multiple repetition of units derived, actually or conceptually, from molecules of low relative molecular mass. Relationships: is a type of regulation of biosynthetic process [GO:0009889]; is a type of regulation of macromolecule metabolic process [GO:0060255]; regulates GO:0009059 Subtypes: GO:0010468, positive regulation of macromolecule biosynthetic process [GO:0010557], negative regulation of macromolecule biosynthetic process [GO:0010558], regulation of glycoprotein biosynthetic process [GO:0010559], regulation of polysaccharide biosynthetic process [GO:0032885], GO:0045113, regulation of MHC class I biosynthetic process [GO:0045343], regulation of MHC class II biosynthetic process [GO:0045346], regulation of hemoglobin biosynthetic process [GO:0046984], GO:0090153, regulation of cutin biosynthetic process [GO:1901957], regulation of protein lipidation [GO:1903059], GO:2000278, regulation of protein geranylgeranylation [GO:2000539], regulation of RNA biosynthetic process [GO:2001141] Sources: GOC:dph, GOC:tb